nuclear-transcribed mRNA catabolic process, 3'-5' exonucleolytic nonsense-mediated decay [GO:0070478] (BP) Definition: The chemical reactions and pathways resulting in the breakdown of the nuclear-transcribed mRNA transcript body of an mRNA in which an amino-acid codon has changed to a nonsense codon; occurs when the 3' end is not protected by a 3'-poly(A) tail; degradation proceeds in the 3' to 5' direction. References: PMID:12769863 Also known as: 3'-5' NMD, 3'-5' nonsense-mediated decay, 3'-5' nonsense-mediated mRNA decay, nuclear-transcribed mRNA breakdown, 3'-5' exonucleolytic nonsense-mediated decay, nuclear-transcribed mRNA catabolism, 3'-5' exonucleolytic nonsense-mediated decay, nuclear-transcribed mRNA degradation, 3'-5' exonucleolytic nonsense-mediated decay Relationships: is a type of nuclear-transcribed mRNA catabolic process, nonsense-mediated decay [GO:0000184]